{
  "gene_name": "Protein kinase C iota type",
  "gene_symbol": "PRKCI",
  "term_id": "GO:0030010",
  "term_label": "establishment of cell polarity",
  "gene": "UniProtKB:P41743"
}